{
  "gene": "UniProtKB:A6H8Z2",
  "gene_name": "Protein FAM221B",
  "term_id": "UNKNOWN:0001",
  "gene_symbol": "FAM221B",
  "term_label": "Unknown molecular function"
}